{
  "gene_symbol": "XPO5",
  "gene": "UniProtKB:Q9HAV4",
  "gene_name": "Exportin-5",
  "term_id": "GO:0005049",
  "term_label": "nuclear export signal receptor activity"
}